coenzyme F420-dependent bicyclic nitroimidazole catabolic process [GO:0052799] (biological process) Also known as: coenzyme F420-dependent nitroimidazole breakdown, coenzyme F420-dependent nitroimidazole catabolism, coenzyme F420-dependent nitroimidazole reduction, coenzyme F420-dependent nitroreductase activity Regulation: regulated by regulation of coenzyme F420-dependent bicyclic nitroimidazole catabolic process [GO:1900288]; RO_0002212 by negative regulation of coenzyme F420-dependent bicyclic nitroimidazole catabolic process [GO:1900289]; positively regulated by positive regulation of coenzyme F420-dependent bicyclic nitroimidazole catabolic process [GO:1900290] Definition: The breakdown of a bicyclic nitroimidazole into simpler components in a process that requires coenzyme F420 and produces reactive nitrogen species. Hydride, from reduced coenzyme F420, is added to the bicyclic nitroimidazole, resulting in unstable substances that break down to form three stable products. The elimination of nitrous acid produces the corresponding des-nitroimidazole; hydrolysis produces a related compound; and further reduction creates an aromatic hydroxylamine metabolite that degrades further. These reactions release hyponitrous acid and nitrous acid, which is unstable and disproportionates into nitric oxide (NO) and other reactive nitrogen intermediates. Relationships: is a type of bicyclic nitroimidazole catabolic process [GO:0052800] References: PMID:16387854, PMID:19039139 Sources: GOC:mengo_curators